cardiac neuron differentiation [GO:0060945] (BP) Definition: The process in which a relatively unspecialized cell acquires specialized features of a neuron of the heart. Sources: GOC:mtg_heart Also known as: heart neuron differentiation Relationships: is a type of cardiocyte differentiation [GO:0035051]; is a type of GO:0048934; is part of autonomic nervous system development [GO:0048483]